{
  "gene_symbol": "RXRB",
  "gene": "UniProtKB:P28702",
  "gene_name": "Retinoic acid receptor RXR-beta",
  "term_id": "GO:0004879",
  "term_label": "nuclear receptor activity"
}